{
  "term_label": "type I interferon-mediated signaling pathway",
  "gene_symbol": "IFNA14",
  "gene": "UniProtKB:P01570",
  "term_id": "GO:0060337",
  "gene_name": "Interferon alpha-14"
}